pronephric glomerulus development [GO:0039021] (biological process) Definition: The progression of the glomerulus of the pronephric kidney over time from its initial formation until its mature state. The pronephric glomerulus is part of the pronephric nephron and is restricted to one body segment. Note: This term is intended for annotation of fish and other organisms which contain a glomerulus as part of the pronephric nephron. It should not be used for annotation of Xenopus, which contains a pronephric glomus rather than a glomerulus. Sources: GOC:dgh, GOC:mtg_kidney_jan10, ZFA:00001557 Relationships: is a type of glomerulus development [GO:0032835]; is part of pronephric nephron development [GO:0039019]